{
  "gene_name": "Protocadherin gamma-A2",
  "gene": "UniProtKB:Q9Y5H1",
  "term_id": "GO:0005886",
  "term_label": "plasma membrane",
  "gene_symbol": "PCDHGA2"
}